fructose:sodium symporter activity [GO:0140930] (MF) Relationships: is a type of GO:0005353; is a type of carbohydrate:monoatomic cation symporter activity [GO:0005402]; is a type of solute:sodium symporter activity [GO:0015370] References: PMID:22212718, PMID:23451068 Definition: Enables the transfer of a solute or solutes from one side of a membrane to the other according to the reaction: D-fructose(out) + Na+(out) = D-fructose(in) + Na+(in).